high-density lipoprotein particle binding [GO:0008035] (molecular function) Definition: Binding to high-density lipoprotein particle, a lipoprotein particle with a high density (typically 1.063-1.21 g/ml) and a diameter of 5-10 nm that contains APOAs and may contain APOCs and APOE. Sources: GOC:mah Also known as: HDL binding Relationships: is a type of GO:0071813